{
  "term_label": "adenylate cyclase-inhibiting G protein-coupled acetylcholine receptor signaling pathway",
  "term_id": "GO:0007197",
  "gene_name": "Muscarinic acetylcholine receptor M4",
  "gene": "UniProtKB:P08173",
  "gene_symbol": "CHRM4"
}